cytidylyltransferase activity [GO:0070567] (molecular function) Relationships: is_a nucleotidyltransferase activity [GO:0016779] Definition: Catalysis of the transfer of a cytidylyl group to an acceptor. Sources: GOC:mah Subtypes: choline-phosphate cytidylyltransferase activity [GO:0004105], GO:0004306, phosphatidate cytidylyltransferase activity [GO:0004605], CCA tRNA nucleotidyltransferase activity [GO:0004810], 3-deoxy-manno-octulosonate cytidylyltransferase activity [GO:0008690], N-acylneuraminate cytidylyltransferase activity [GO:0008781], GO:0043338, glucose-1-phosphate cytidylyltransferase activity [GO:0047343], glycerol-3-phosphate cytidylyltransferase activity [GO:0047348], D-ribitol-5-phosphate cytidylyltransferase activity [GO:0047349], GO:0047353, 2-C-methyl-D-erythritol 4-phosphate cytidylyltransferase activity [GO:0050518], CC tRNA cytidylyltransferase activity [GO:0052927], GO:0061602, N-glycolylneuraminic acid (Neu5Gc) cytidylyltransferase activity [GO:0090632], keto-deoxynonulosonic acid (KDN) cytidylyltransferase activity [GO:0090633], CCACCA tRNA nucleotidyltransferase activity [GO:0160016]